septin band [GO:0032158] (cellular component) Definition: A diffuse ring composed of a series of septin bars that run parallel to the long axis of the cell. This type of septin structure has been observed in a number of locations associated with polarized grown and/or deposition of new membrane, but not with cytokinesis, such as at the shmoo (mating projection) neck, at the junction between the mother cell and the germ tube (hypha) of a fungal cell growing filamentously. Relationships: is a type of cellular anatomical structure [GO:0110165]; is part of septin cytoskeleton [GO:0032156] Subtypes: mating projection septin band [GO:0032162], GO:0032163 References: PMID:16151244 Sources: GOC:krc